{
  "term_id": "GO:0071339",
  "gene": "UniProtKB:Q9NXF1",
  "gene_symbol": "TEX10",
  "gene_name": "Testis-expressed protein 10",
  "term_label": "MLL1 complex"
}